metanephric cap specification [GO:0072188] (biological process) Relationships: is a type of renal system pattern specification [GO:0072048]; is a type of metanephric cap formation [GO:0072187]; is_a GO:0072268 Definition: The process in which the metanephric cap acquires its identity. Sources: GOC:mtg_kidney_jan10